{
  "gene_name": "E3 ubiquitin-protein ligase ZNRF2",
  "gene_symbol": "ZNRF2",
  "term_id": "GO:0043161",
  "gene": "UniProtKB:Q8NHG8",
  "term_label": "proteasome-mediated ubiquitin-dependent protein catabolic process"
}